{
  "gene_symbol": "HCRT",
  "term_id": "GO:0005184",
  "gene_name": "Hypocretin neuropeptide precursor",
  "term_label": "neuropeptide hormone activity",
  "gene": "UniProtKB:O43612"
}